{
  "term_label": "synaptic signaling",
  "term_id": "GO:0099536",
  "gene_name": "Dystrophin-related protein 2",
  "gene": "UniProtKB:Q13474",
  "gene_symbol": "DRP2"
}